L-fucose mutarotase activity [GO:0036373] (molecular function) Definition: Catalysis of the reaction: alpha-L-fucose = beta-L-fucose. Also known as: alpha-L-fucose 1-epimerase activity, fucose 1-epimerase activity, type-2 mutarotase activity Relationships: is a type of racemase and epimerase activity, acting on carbohydrates and derivatives [GO:0016857] References: PMID:15060078 Sources: GOC:crds, RHEA:25580